{
  "gene_name": "Arylsulfatase B",
  "term_id": "UNKNOWN:0003",
  "gene": "UniProtKB:P15848",
  "gene_symbol": "ARSB",
  "term_label": "Unknown cellular component"
}